{
  "gene": "UniProtKB:O60858",
  "gene_name": "E3 ubiquitin-protein ligase TRIM13",
  "term_id": "GO:0036503",
  "term_label": "ERAD pathway",
  "gene_symbol": "TRIM13"
}